{
  "gene_symbol": "PSAP",
  "gene": "UniProtKB:P07602",
  "gene_name": "Prosaposin",
  "term_id": "GO:0005615",
  "term_label": "extracellular space"
}